{
  "gene": "UniProtKB:Q9UN71",
  "gene_symbol": "PCDHGB4",
  "term_label": "plasma membrane",
  "term_id": "GO:0005886",
  "gene_name": "Protocadherin gamma-B4"
}